regulation of homotypic cell-cell adhesion [GO:0034110] (biological process) Definition: Any process that modulates the frequency, rate, or extent of homotypic cell-cell adhesion. Subtypes: GO:0034111, positive regulation of homotypic cell-cell adhesion [GO:0034112], regulation of erythrocyte aggregation [GO:0034118], regulation of platelet aggregation [GO:0090330] Sources: GOC:add Relationships: is a type of regulation of cell-cell adhesion [GO:0022407]; regulates GO:0034109